regulation of sister chromatid cohesion [GO:0007063] (biological process) Sources: GOC:go_curators Subtypes: regulation of maintenance of sister chromatid cohesion [GO:0034091], GO:0045875, GO:0045876, regulation of centromeric sister chromatid cohesion [GO:0070602] Relationships: is a type of GO:0010564; is a type of regulation of chromosome organization [GO:0033044]; RO_0002211 GO:0007062 Definition: Any process that modulates the frequency, rate or extent of sister chromatid cohesion.